{
  "gene_name": "Pre-B-cell leukemia transcription factor 2",
  "term_id": "GO:0048568",
  "gene_symbol": "PBX2",
  "gene": "UniProtKB:P40425",
  "term_label": "embryonic organ development"
}